{
  "gene": "UniProtKB:Q96LX8",
  "term_id": "GO:0000978",
  "gene_symbol": "ZNF597",
  "term_label": "RNA polymerase II cis-regulatory region sequence-specific DNA binding",
  "gene_name": "Zinc finger protein 597"
}